{
  "gene_symbol": "VANGL2",
  "term_id": "GO:0060071",
  "term_label": "Wnt signaling pathway, planar cell polarity pathway",
  "gene": "UniProtKB:Q9ULK5",
  "gene_name": "Vang-like protein 2"
}